negative regulation of arachidonate secretion [GO:1900139] (biological process) Relationships: is a type of negative regulation of icosanoid secretion [GO:0032304]; is a type of regulation of arachidonate secretion [GO:0090237]; negatively regulates arachidonate secretion [GO:0050482] Sources: GOC:TermGenie Definition: Any process that stops, prevents or reduces the frequency, rate or extent of arachidonic acid secretion. Also known as: down regulation of arachidonic acid secretion, down-regulation of arachidonic acid secretion, downregulation of arachidonic acid secretion, negative regulation of arachidonic acid secretion, inhibition of arachidonic acid secretion